ESCRT III complex disassembly [GO:1904903] (biological process) Definition: The disaggregation of an ESCRT III complex into its constituent components. References: PMID:20588296 Sources: GOC:PARL, GOC:TermGenie, GOC:pad, GO_REF:0000079 Relationships: is a type of GO:1904896